{
  "gene_symbol": "HBD",
  "gene_name": "Hemoglobin subunit delta",
  "gene": "UniProtKB:P02042",
  "term_label": "oxygen carrier activity",
  "term_id": "GO:0005344"
}